{
  "term_label": "Unknown cellular component",
  "term_id": "UNKNOWN:0003",
  "gene_symbol": "RNF214",
  "gene_name": "RING finger protein 214",
  "gene": "UniProtKB:Q8ND24"
}